regulation protein catabolic process at postsynapse [GO:0140252] (biological process) Relationships: is a type of regulation protein catabolic process at synapse [GO:0140250]; occurs in GO:0098794 Definition: Any process that modulates the frequency, rate or extent of the chemical reactions and pathways resulting in the breakdown of a protein at the postsynapse. References: PMID:17062563 Note: Note that this term was created for the SynGO project, and will be obsoleted when the SynGO annotations are made in Noctua.